{
  "term_label": "ubiquitin-like protein binding",
  "term_id": "GO:0032182",
  "gene_symbol": "DCUN1D5",
  "gene": "UniProtKB:Q9BTE7",
  "gene_name": "DCN1-like protein 5"
}